{
  "term_label": "regulation of transcription by RNA polymerase II",
  "term_id": "GO:0006357",
  "gene": "UniProtKB:Q8NEK5",
  "gene_symbol": "ZNF548",
  "gene_name": "Zinc finger protein 548"
}